ring centriole [GO:0061823] (cellular component) Definition: A ring-like structure observed at the base of the ciliary cap of insect spermatids. This structure may anchor the axoneme to the ciliary cap membrane and/or act as a diffusion barrier, proposed to be analogous to the annulus of mammalian sperm flagellum. References: PMID:25447994, PMID:4903810 Relationships: is a type of cellular anatomical structure [GO:0110165]; is part of cilium [GO:0005929]